cellular response to acetate [GO:0071311] (biological process) Sources: GOC:mah Definition: Any process that results in a change in state or activity of a cell (in terms of movement, secretion, enzyme production, gene expression, etc.) as a result of an acetate stimulus. Relationships: is a type of response to acetate [GO:0010034]; is a type of cellular response to oxygen-containing compound [GO:1901701]